oxidised low-density lipoprotein particle clearance [GO:0150024] (biological process) Definition: The process in which an oxidised low-density lipoprotein particle is removed from the blood via receptor-mediated endocytosis and its constituent parts degraded. References: PMID:27607416 Sources: GOC:aruk, GOC:bc Also known as: ox-LDL particle clearance, oxLDL particle clearance, oxidised LDL particle clearance, oxidized LDL particle clearance, oxidized low-density lipoprotein particle clearance Relationships: is a type of plasma lipoprotein particle clearance [GO:0034381]